{
  "gene": "UniProtKB:P78536",
  "gene_symbol": "ADAM17",
  "gene_name": "Disintegrin and metalloproteinase domain-containing protein 17",
  "term_label": "membrane protein ectodomain proteolysis",
  "term_id": "GO:0006509"
}